anatomical structure development [GO:0048856] (biological process) Also known as: development of an anatomical structure Relationships: is_a GO:0032502 Sources: GO_REF:0000021 Subtypes: ovarian follicle development [GO:0001541], blood vessel development [GO:0001568], insect visual primordium development [GO:0001748], blastocyst development [GO:0001824], maternal placenta development [GO:0001893], hair follicle development [GO:0001942], lymph vessel development [GO:0001945], GO:0002088, endocardium development [GO:0003157], heart valve development [GO:0003170], cardiac chamber development [GO:0003205], cardiac septum development [GO:0003279], brainstem development [GO:0003360], neural retina development [GO:0003407], anterior rotation of the optic cup [GO:0003410], multicellular organism development [GO:0007275], ventral midline development [GO:0007418], GO:0007458, notum development [GO:0007477], GO:0007487, anterior midgut development [GO:0007496], GO:0007497, tissue development [GO:0009888], suspensor development [GO:0010098], seed coat development [GO:0010214], GO:0010254, stipule development [GO:0010865], mushroom body development [GO:0016319], dendrite development [GO:0016358], GO:0021510, dorsal spinal cord development [GO:0021516], ventral spinal cord development [GO:0021517], diencephalon development [GO:0021536], telencephalon development [GO:0021537], epithalamus development [GO:0021538], subthalamus development [GO:0021539], ammon gyrus development [GO:0021541], dentate gyrus development [GO:0021542], pallium development [GO:0021543], subpallium development [GO:0021544], rhombomere development [GO:0021546], GO:0021548, cerebellum development [GO:0021549], medulla oblongata development [GO:0021550], fourth ventricle development [GO:0021592], lateral ventricle development [GO:0021670], GO:0021675, third ventricle development [GO:0021678], cerebellar molecular layer development [GO:0021679], GO:0021680, GO:0021681, cerebellar cortex development [GO:0021695], medullary reticular formation development [GO:0021723], intermediate reticular formation development [GO:0021727], superior reticular formation development [GO:0021729], striatum development [GO:0021756], amygdala development [GO:0021764], cingulate gyrus development [GO:0021765], hippocampus development [GO:0021766], mammillary body development [GO:0021767], orbitofrontal cortex development [GO:0021769], parahippocampal gyrus development [GO:0021770], GO:0021772, thalamus development [GO:0021794], hypothalamus development [GO:0021854], forebrain-midbrain boundary formation [GO:0021905], adenohypophysis development [GO:0021984], GO:0021986, cerebral cortex development [GO:0021987], GO:0021988, olfactory cortex development [GO:0021989], GO:0022037, GO:0022038, forebrain development [GO:0030900], midbrain development [GO:0030901], hindbrain development [GO:0030902], GO:0030917, endocrine pancreas development [GO:0031018], regeneration [GO:0031099], glomerulus development [GO:0032835], GO:0032836, floor plate development [GO:0033504], tube development [GO:0035295], adrenal cortex development [GO:0035801], cloaca development [GO:0035844], nail development [GO:0035878], ascending aorta development [GO:0035905], GO:0035906, deltoid tuberosity development [GO:0035993], atrioventricular canal development [GO:0036302], embryonic heart tube elongation [GO:0036306], GO:0039009, GO:0039012, nephrostome development [GO:0039018], cuticle development [GO:0042335], tooth eruption [GO:0044691], GO:0048036, compound eye corneal lens development [GO:0048058], GO:0048098, germ-line cyst encapsulation [GO:0048138], lung alveolus development [GO:0048286], mesendoderm development [GO:0048382], floral whorl development [GO:0048438], cell development [GO:0048468], style development [GO:0048479], GO:0048480, animal organ development [GO:0048513], GO:0048608, anther development [GO:0048653], anther wall tapetum development [GO:0048658], GO:0048722, clypeus development [GO:0048723], GO:0048724, labrum development [GO:0048726], posterior cibarial plate development [GO:0048727], system development [GO:0048731], appendage development [GO:0048736], root cap development [GO:0048829], inner ear development [GO:0048839], otolith development [GO:0048840], neural nucleus development [GO:0048857], GO:0048868, cupula development [GO:0048887], GO:0060021, hard palate development [GO:0060022], GO:0060023, GO:0060041, olfactory pit development [GO:0060166], GO:0060322, face development [GO:0060324], lung saccule development [GO:0060430], lung lobe development [GO:0060462], pharynx development [GO:0060465], prostate glandular acinus development [GO:0060525], GO:0060618, labyrinthine layer development [GO:0060711], mammary gland alveolus development [GO:0060749], dendritic spine development [GO:0060996], umbilical cord development [GO:0061027], eyelid development in camera-type eye [GO:0061029], GO:0061032, olfactory bulb mitral cell layer development [GO:0061034], dermatome development [GO:0061054], myotome development [GO:0061055], GO:0061061, left horn of sinus venosus development [GO:0061079], right horn of sinus venosus development [GO:0061080], GO:0061152, fungiform papilla development [GO:0061196], GO:0061303, GO:0061360, mammillary axonal complex development [GO:0061373], GO:0061374, mammillotectal axonal tract development [GO:0061375], mammillotegmental axonal tract development [GO:0061376], GO:0061377, corpora quadrigemina development [GO:0061378], inferior colliculus development [GO:0061379], superior colliculus development [GO:0061380], central canal development [GO:0061524], stomach development [GO:0062094], Kupffer's vesicle development [GO:0070121], GO:0070788, superior temporal gyrus development [GO:0071109], ectodermal placode development [GO:0071696], beak development [GO:0071728], nephron development [GO:0072006], glomus development [GO:0072013], descending thin limb development [GO:0072022], GO:0072051, renal inner medulla development [GO:0072053], GO:0072054, renal cortex development [GO:0072055], pyramid development [GO:0072056], inner stripe development [GO:0072057], outer stripe development [GO:0072058], cortical collecting duct development [GO:0072059], vascular cord development [GO:0072360], germ tube formation [GO:0075009], stamen filament development [GO:0080086], stomium development [GO:0080166], GO:0090102, aerial mycelium formation [GO:0097736], substrate mycelium formation [GO:0097738], socially cooperative development [GO:0099120], GO:0099402, yolk syncytial layer development [GO:0106336], cutin-based cuticle development [GO:0160062], caecum development [GO:1903700], substantia propria of cornea development [GO:1903701], esophagus development [GO:1903702], palisade mesophyll development [GO:1903866], GO:1903867, serous membrane development [GO:1904817], visceral peritoneum development [GO:1904818], GO:1904819, GO:1904866, cranial skeletal system development [GO:1904888], plant septum development [GO:1905328], sclerotium development [GO:1990045], fruit replum development [GO:1990058], GO:1990059 Definition: The biological process whose specific outcome is the progression of an anatomical structure from an initial condition to its mature state. This process begins with the formation of the structure and ends with the mature structure, whatever form that may be including its natural destruction. An anatomical structure is any biological entity that occupies space and is distinguished from its surroundings. Anatomical structures can be macroscopic such as a carpel, or microscopic such as an acrosome.